{
  "term_id": "GO:0006888",
  "gene_name": "Protein TFG",
  "term_label": "endoplasmic reticulum to Golgi vesicle-mediated transport",
  "gene": "UniProtKB:Q92734",
  "gene_symbol": "TFG"
}